{
  "gene_symbol": "SAPCD1",
  "gene": "UniProtKB:Q5SSQ6",
  "term_id": "UNKNOWN:0001",
  "gene_name": "Suppressor APC domain-containing protein 1",
  "term_label": "Unknown molecular function"
}